nitrate:proton symporter activity [GO:0009671] (molecular function) References: PMID:10066586, PMID:1990981 Sources: GOC:mah Relationships: is a type of GO:0015295; is a type of high-affinity secondary active nitrite transmembrane transporter activity [GO:0015513] Definition: Enables the transfer of a solute or solutes from one side of a membrane to the other according to the reaction: nitrate(out) + H+(out) = nitrate(in) + H+(in). Also known as: nitrate(chlorate):hydrogen symporter activity, nitrate(chlorate):proton symporter activity, nitrate:hydrogen symporter activity